{
  "gene_symbol": "OGFOD3",
  "gene": "UniProtKB:Q6PK18",
  "term_id": "UNKNOWN:0003",
  "gene_name": "2-oxoglutarate and iron-dependent oxygenase domain-containing protein 3",
  "term_label": "Unknown cellular component"
}